{
  "gene": "UniProtKB:Q6UB35",
  "gene_name": "Monofunctional C1-tetrahydrofolate synthase, mitochondrial",
  "term_label": "formate-tetrahydrofolate ligase activity",
  "gene_symbol": "MTHFD1L",
  "term_id": "GO:0004329"
}